{
  "term_label": "olfactory receptor activity",
  "gene_symbol": "OR5B21",
  "gene_name": "Olfactory receptor 5B21",
  "gene": "UniProtKB:A6NL26",
  "term_id": "GO:0004984"
}